{
  "gene_name": "Acetyl-coenzyme A thioesterase",
  "gene": "UniProtKB:Q8WYK0",
  "term_label": "cytoplasm",
  "term_id": "GO:0005737",
  "gene_symbol": "ACOT12"
}